{
  "gene_name": "Fibrillin-2",
  "term_id": "GO:0005179",
  "gene_symbol": "FBN2",
  "gene": "UniProtKB:P35556",
  "term_label": "hormone activity"
}